{
  "gene": "UniProtKB:Q6ZQX7",
  "term_id": "GO:0005730",
  "gene_symbol": "LIAT1",
  "term_label": "nucleolus",
  "gene_name": "Protein LIAT1"
}